{
  "gene_name": "TLC domain-containing protein 1",
  "gene_symbol": "TLCD1",
  "term_id": "GO:0071709",
  "gene": "UniProtKB:Q96CP7",
  "term_label": "membrane assembly"
}